{
  "gene": "UniProtKB:P23471",
  "gene_name": "Receptor-type tyrosine-protein phosphatase zeta",
  "term_id": "GO:0007165",
  "term_label": "signal transduction",
  "gene_symbol": "PTPRZ1"
}